negative regulation of pseurotin A biosynthetic process [GO:1900850] (biological process) Also known as: down regulation of pseurotin A biosynthetic process, down-regulation of pseurotin A biosynthetic process, downregulation of pseurotin A biosynthetic process Definition: Any process that stops, prevents or reduces the frequency, rate or extent of pseurotin A biosynthetic process. Sources: GOC:TermGenie, GOC:di Relationships: is a type of GO:0009890; is a type of negative regulation of amide metabolic process [GO:0034249]; is_a GO:0062014; is a type of GO:1900849; RO_0002212 pseurotin A biosynthetic process [GO:1900790]